{
  "gene_symbol": "A0A7P0T9M0",
  "term_id": "UNKNOWN:0001",
  "gene_name": "Uncharacterized protein",
  "term_label": "Unknown molecular function",
  "gene": "UniProtKB:A0A7P0T9M0"
}